activation of Janus kinase activity [GO:0042976] (biological process) References: PMID:12479803 Sources: GOC:jl Also known as: activation of JAK protein, activation of JAK protein by tyrosine phosphorylation, positive regulation of JAK protein activity by tyrosine phosphorylation, tyrosine phosphorylation of JAK protein, activation of JAK1 kinase activity, activation of JAK1 protein, activation of JAK2 kinase activity, activation of JAK2 protein, tyrosine phosphorylation of JAK1 protein, tyrosine phosphorylation of JAK2 protein Relationships: is a type of peptidyl-tyrosine phosphorylation [GO:0018108]; is a type of activation of protein kinase activity [GO:0032147]; is part of GO:0046427 Definition: The process of introducing a phosphate group to a tyrosine residue of a JAK (Janus Activated Kinase) protein, thereby activating it.